{
  "term_label": "central nervous system neuron differentiation",
  "gene_name": "Nuclear receptor subfamily 4 group A member 2",
  "gene_symbol": "NR4A2",
  "term_id": "GO:0021953",
  "gene": "UniProtKB:P43354"
}